{
  "term_id": "GO:0005886",
  "gene_symbol": "OR1A1",
  "gene": "UniProtKB:Q9P1Q5",
  "gene_name": "Olfactory receptor 1A1",
  "term_label": "plasma membrane"
}